cellular component organization [GO:0016043] (biological process) Regulation: regulated by GO:0051128; negatively regulated by negative regulation of cellular component organization [GO:0051129]; positively regulated by GO:0051130 Also known as: cell organisation, cellular component organisation at cellular level, cellular component organisation in other organism, cellular component organization at cellular level, cellular component organization in other organism, cell organization and biogenesis Relationships: is a type of cellular component organization or biogenesis [GO:0071840] Subtypes: chromatin organization [GO:0006325], organelle organization [GO:0006996], GO:0007028, endomembrane system organization [GO:0010256], cellular component disassembly [GO:0022411], cellular component assembly [GO:0022607], cell projection organization [GO:0030030], GO:0031023, oral apparatus organization [GO:0032122], regulation of cellular component size [GO:0032535], cellular anatomical entity morphogenesis [GO:0032989], cell junction organization [GO:0034330], microtubule organizing center attachment site organization [GO:0034994], GO:0035845, extracellular structure organization [GO:0043062], periplasmic space organization [GO:0043580], protein-containing complex organization [GO:0043933], cellular component maintenance [GO:0043954], actin cortical patch organization [GO:0044396], external encapsulating structure organization [GO:0045229], membrane organization [GO:0061024], blood microparticle formation [GO:0072564], plastoglobule organization [GO:0080177], supramolecular fiber organization [GO:0097435], vesicle tethering [GO:0099022], presynapse organization [GO:0099172], postsynapse organization [GO:0099173], cilium attachment to cell body [GO:0120309], GO:0160194, post-anaphase microtubule array organization [GO:1904186], mitochondrion-endoplasmic reticulum membrane tethering [GO:1990456], presynaptic active zone organization [GO:1990709], vacuole-ER tethering [GO:1990854] Definition: A process that results in the assembly, arrangement of constituent parts, or disassembly of a cellular component. Sources: GOC:ai, GOC:jl, GOC:mah